{
  "gene_symbol": "TRAJ16",
  "gene_name": "T cell receptor alpha joining 16 (Fragment)",
  "term_id": "UNKNOWN:0003",
  "gene": "UniProtKB:A0A075B6V0",
  "term_label": "Unknown cellular component"
}